{
  "gene_symbol": "TMEM151A",
  "term_label": "membrane",
  "gene": "UniProtKB:Q8N4L1",
  "term_id": "GO:0016020",
  "gene_name": "Transmembrane protein 151A"
}